{
  "gene_symbol": "DEFB115",
  "term_label": "killing of cells of another organism",
  "term_id": "GO:0031640",
  "gene_name": "Beta-defensin 115",
  "gene": "UniProtKB:Q30KQ5"
}